{
  "gene": "UniProtKB:Q9HB14",
  "gene_symbol": "KCNK13",
  "term_label": "potassium ion transmembrane transport",
  "term_id": "GO:0071805",
  "gene_name": "Potassium channel subfamily K member 13"
}